fluoride transmembrane transporter activity [GO:1903425] (molecular function) Definition: Enables the transfer of fluoride from one side of a membrane to the other. Relationships: is_a monoatomic anion transmembrane transporter activity [GO:0008509]; is part of fluoride transmembrane transport [GO:1903424] References: PMID:24173035 Sources: GOC:TermGenie, GO_REF:0000070 Subtypes: fluoride channel activity [GO:0062054]